{
  "term_id": "GO:0005669",
  "gene_symbol": "LINC02218",
  "term_label": "transcription factor TFIID complex",
  "gene": "UniProtKB:A0A1W2PRN6",
  "gene_name": "HCG1807616"
}